{
  "term_id": "GO:0030280",
  "gene_name": "Keratin, type II cytoskeletal 80",
  "gene_symbol": "KRT80",
  "term_label": "structural constituent of skin epidermis",
  "gene": "UniProtKB:Q6KB66"
}